{
  "gene": "UniProtKB:P51530",
  "term_label": "5'-flap endonuclease activity",
  "gene_symbol": "DNA2",
  "term_id": "GO:0017108",
  "gene_name": "DNA replication ATP-dependent helicase_nuclease DNA2"
}